{
  "term_label": "N-acetylglucosamine kinase activity",
  "gene_symbol": "NAGK",
  "gene_name": "N-acetyl-D-glucosamine kinase",
  "term_id": "GO:0045127",
  "gene": "UniProtKB:Q9UJ70"
}